{
  "gene": "UniProtKB:Q7Z2D5",
  "gene_symbol": "PLPPR4",
  "term_label": "plasma membrane",
  "gene_name": "Phospholipid phosphatase-related protein type 4",
  "term_id": "GO:0005886"
}